{
  "gene_name": "Protein arginine methyltransferase NDUFAF7, mitochondrial",
  "term_id": "GO:0005739",
  "term_label": "mitochondrion",
  "gene": "UniProtKB:Q7L592",
  "gene_symbol": "NDUFAF7"
}